cyclin L-CDK11 complex [GO:0180038] (cellular component) Also known as: Cdk11-Cyclin L complex References: PMID:23122962, PMID:32446654 Relationships: is a type of cyclin-dependent protein kinase holoenzyme complex [GO:0000307] Definition: A protein complex consisting of cyclin L and cyclin-dependent kinase 11 (CDK11). Cyclins are characterized by periodicity in protein abundance throughout the cell cycle. Cyclin-dependent kinases represent a family of serine/threonine protein kinases that become active upon binding to a cyclin regulatory partner.